{
  "gene_name": "Fibrillin-2",
  "gene_symbol": "FBN2",
  "term_label": "extracellular region",
  "gene": "UniProtKB:P35556",
  "term_id": "GO:0005576"
}